{
  "term_id": "GO:0003899",
  "gene_name": "DNA-directed RNA polymerases I, II, and III subunit RPABC2",
  "gene": "UniProtKB:P61218",
  "gene_symbol": "POLR2F",
  "term_label": "DNA-directed RNA polymerase activity"
}